{
  "term_id": "GO:0033622",
  "gene_symbol": "FERMT3",
  "term_label": "integrin activation",
  "gene_name": "Fermitin family homolog 3",
  "gene": "UniProtKB:Q86UX7"
}